IRE1-mediated unfolded protein response [GO:0036498] (biological process) References: PMID:22013210 Sources: GOC:PARL, GOC:bf Note: Consider also annotating to 'eiF2alpha phosphorylation in response to endoplasmic reticulum stress ; GO:0036492' or its descendants. Definition: The series of molecular signals mediated by the endoplasmic reticulum stress sensor IRE1 (Inositol-requiring transmembrane kinase/endonuclease). Begins with activation of IRE1 in response to endoplasmic reticulum (ER) stress, and ends with regulation of a downstream cellular process, e.g. transcription. One target of activated IRE1 is the transcription factor HAC1 in yeast, or XBP1 in mammals; IRE1 cleaves an intron of a mRNA coding for HAC1/XBP1 to generate an activated HAC1/XBP1 transcription factor, which controls the up regulation of UPR-related genes. At least in mammals, IRE1 can also signal through additional intracellular pathways including JNK and NF-kappaB. Regulation: regulated by GO:1903894; RO_0002212 by negative regulation of IRE1-mediated unfolded protein response [GO:1903895]; RO_0002213 by positive regulation of IRE1-mediated unfolded protein response [GO:1903896] Also known as: IRE1 signal transduction pathway, IRE1 branch of UPR, UPR signaling by IRE1 stress sensor, endoplasmic reticulum unfolded protein response; IRE1 signaling, IRE1alpha unfolded protein response, IRE1p unfolded protein response, ERN1-mediated unfolded protein response, IRE1 signaling in response to endoplasmic reticulum stress, inositol-requiring enzyme 1-mediated unfolded protein response, inositol-requiring transmembrane kinase/endonuclease signal transduction Relationships: is a type of endoplasmic reticulum unfolded protein response [GO:0030968]